regulation of plant organ morphogenesis [GO:1905421] (biological process) Definition: Any process that modulates the frequency, rate or extent of plant organ morphogenesis. Subtypes: regulation of leaf morphogenesis [GO:1901371], negative regulation of plant organ morphogenesis [GO:1905422], positive regulation of plant organ morphogenesis [GO:1905423], regulation of root morphogenesis [GO:2000067] Relationships: is_a regulation of anatomical structure morphogenesis [GO:0022603]; regulates GO:1905392 Sources: GOC:TermGenie, GOC:tb, GO_REF:0000058